{
  "gene_symbol": "TCIM",
  "term_label": "endothelial cell activation involved in immune response",
  "gene_name": "Transcriptional and immune response regulator",
  "term_id": "GO:0002264",
  "gene": "UniProtKB:Q9NR00"
}